{
  "term_label": "phosphatidylcholine metabolic process",
  "term_id": "GO:0046470",
  "gene_symbol": "PLA2G2C",
  "gene": "UniProtKB:Q5R387",
  "gene_name": "Putative inactive group IIC secretory phospholipase A2"
}